versiconal hemiacetal acetate reductase activity [GO:0102975] (molecular function) Relationships: is a type of oxidoreductase activity, acting on the CH-OH group of donors, NAD or NADP as acceptor [GO:0016616] Definition: Catalysis of the reaction: versiconol acetate + NADP = versiconal hemiacetal acetate + NADPH. Sources: RHEA:35695